regulation of cAMP/PKA signal transduction [GO:0141161] (biological process) Sources: GOC:curators Relationships: is a type of regulation of intracellular signal transduction [GO:1902531]; regulates GO:0141156 Definition: Any process that modulates the frequency, rate or extent of cAMP/PKA signal transduction. Subtypes: negative regulation of cAMP/PKA signal transduction [GO:0141162], positive regulation of cAMP/PKA signal transduction [GO:0141163] Also known as: regulation of cAMP/PKA signaling